{
  "gene": "UniProtKB:Q16740",
  "gene_name": "ATP-dependent Clp protease proteolytic subunit, mitochondrial",
  "gene_symbol": "CLPP",
  "term_id": "GO:0051117",
  "term_label": "ATPase binding"
}